{
  "term_label": "Unknown cellular component",
  "term_id": "UNKNOWN:0003",
  "gene_name": "C1GALT1-specific chaperone 1",
  "gene_symbol": "C1GALT1C1",
  "gene": "UniProtKB:Q96EU7"
}